{
  "term_id": "UNKNOWN:0003",
  "gene_name": "DNA endonuclease RBBP8",
  "term_label": "Unknown cellular component",
  "gene_symbol": "RBBP8",
  "gene": "UniProtKB:Q99708"
}